{
  "gene_symbol": "VKORC1",
  "gene_name": "Vitamin K epoxide reductase complex subunit 1",
  "gene": "UniProtKB:Q9BQB6",
  "term_label": "vitamin K metabolic process",
  "term_id": "GO:0042373"
}